{
  "gene": "UniProtKB:P27169",
  "gene_symbol": "PON1",
  "gene_name": "Serum paraoxonase_arylesterase 1",
  "term_label": "extracellular space",
  "term_id": "GO:0005615"
}